negative regulation of dipeptide transmembrane transport [GO:2001149] (biological process) Also known as: negative regulation of dipeptide membrane transport Definition: Any process that stops, prevents or reduces the frequency, rate or extent of dipeptide transmembrane transport. Sources: GOC:obol Relationships: is a type of negative regulation of transmembrane transport [GO:0034763]; is a type of negative regulation of dipeptide transport [GO:2000879]; is a type of regulation of dipeptide transmembrane transport [GO:2001148]; negatively regulates dipeptide transmembrane transport [GO:0035442]